{
  "gene": "UniProtKB:Q6YI46",
  "gene_symbol": "TMEM64",
  "term_id": "GO:0005783",
  "term_label": "endoplasmic reticulum",
  "gene_name": "Transmembrane protein 64"
}